{
  "gene_symbol": "ZIC5",
  "gene": "UniProtKB:Q96T25",
  "term_id": "GO:0007417",
  "gene_name": "Zinc finger protein ZIC 5",
  "term_label": "central nervous system development"
}